{
  "term_label": "Unknown biological process",
  "gene": "UniProtKB:A0A0A0MT84",
  "term_id": "UNKNOWN:0002",
  "gene_name": "T cell receptor gamma joining P2 (Fragment)",
  "gene_symbol": "TRGJP2"
}